{
  "gene_name": "HLA class I histocompatibility antigen, A alpha chain",
  "term_id": "GO:0002486",
  "gene": "UniProtKB:P04439",
  "term_label": "antigen processing and presentation of endogenous peptide antigen via MHC class I via ER pathway, TAP-independent",
  "gene_symbol": "HLA-A"
}